{
  "gene_symbol": "GLP2R",
  "gene_name": "Glucagon-like peptide 2 receptor",
  "gene": "UniProtKB:O95838",
  "term_id": "GO:0005886",
  "term_label": "plasma membrane"
}